carbon tetrachloride catabolic process [GO:0019382] (biological process) Definition: The chemical reactions and pathways resulting in the breakdown of carbon tetrachloride, a toxic, carcinogenic compound which is used as a general solvent in industrial degreasing operations. It is also used as grain fumigant and a chemical intermediate in the production of refrigerants. Relationships: is a type of GO:0018885; is_a halogenated hydrocarbon catabolic process [GO:0042206] Also known as: carbon tetrachloride breakdown, carbon tetrachloride catabolism, carbon tetrachloride degradation Sources: GOC:go_curators